{
  "term_id": "GO:0000978",
  "gene_symbol": "PBX3",
  "gene_name": "Pre-B-cell leukemia transcription factor 3",
  "term_label": "RNA polymerase II cis-regulatory region sequence-specific DNA binding",
  "gene": "UniProtKB:P40426"
}